primary amine secretion, neurotransmission [GO:0061532] (biological process) Sources: GOC:dph Definition: The regulated release of a primary amine by a cell, in which the primary amine acts as a neurotransmitter. Relationships: is a type of neurotransmitter secretion [GO:0007269]; is a type of GO:0061531 Subtypes: tyramine secretion, neurotransmission [GO:0061546]